{
  "gene_name": "Putative uncharacterized protein FLJ36797",
  "term_label": "Unknown molecular function",
  "gene_symbol": "Q8N9P0",
  "term_id": "UNKNOWN:0001",
  "gene": "UniProtKB:Q8N9P0"
}